{
  "term_label": "triglyceride biosynthetic process",
  "gene_symbol": "GPAM",
  "term_id": "GO:0019432",
  "gene": "UniProtKB:Q9HCL2",
  "gene_name": "Glycerol-3-phosphate acyltransferase 1, mitochondrial"
}